{
  "gene_name": "Regulatory factor X-associated protein",
  "term_label": "regulation of transcription by RNA polymerase II",
  "gene_symbol": "RFXAP",
  "term_id": "GO:0006357",
  "gene": "UniProtKB:O00287"
}